{
  "gene": "UniProtKB:P50607",
  "gene_symbol": "TUB",
  "gene_name": "Tubby protein homolog",
  "term_label": "cilium",
  "term_id": "GO:0005929"
}